regulation of telomere maintenance [GO:0032204] (biological process) Definition: Any process that modulates the frequency, rate or extent of a process that affects and monitors the activity of telomeric proteins and the length of telomeric DNA. Sources: GOC:mah Relationships: is a type of GO:0033044; is a type of regulation of DNA metabolic process [GO:0051052]; regulates telomere maintenance [GO:0000723] Subtypes: negative regulation of telomere maintenance [GO:0032205], positive regulation of telomere maintenance [GO:0032206], regulation of telomere maintenance via recombination [GO:0032207], GO:0032213, regulation of telomere capping [GO:1904353], GO:1904356, GO:1904418, regulation of t-circle formation [GO:1904429], GO:1904505, regulation of telomeric loop disassembly [GO:1904533]